protein serine kinase activity (using GTP as donor) [GO:0106264] (molecular function) References: PMID:32322062 Sources: GOC:sp, RHEA:64020 Relationships: is a type of protein kinase activity [GO:0004672] Definition: Catalysis of the reactions: GTP + L-seryl-[protein] = GDP + H+ + O-phospho-L-seryl-[protein].